histamine secretion mediated by immunoglobulin [GO:0097280] (biological process) References: PMID:11490155, PMID:1719184 Sources: GOC:add, GOC:rv Relationships: is a type of GO:0002437; is a type of GO:0002441; is_a response to histamine [GO:0034776]; has part antigen binding [GO:0003823] Subtypes: histamine secretion mediated by IgE immunoglobulin [GO:0097279] Definition: Histamine release triggered by the binding of an antigen to an immunoglobulin bound to the cell surface.